{
  "term_id": "GO:0005634",
  "term_label": "nucleus",
  "gene": "UniProtKB:Q86Z02",
  "gene_name": "Homeodomain-interacting protein kinase 1",
  "gene_symbol": "HIPK1"
}